interleukin-5 binding [GO:0019980] (molecular function) Definition: Binding to interleukin-5. Sources: GOC:jl Also known as: IL-5 binding Relationships: is a type of growth factor binding [GO:0019838]; is a type of cytokine binding [GO:0019955]